{
  "gene": "UniProtKB:Q9H2J4",
  "term_label": "cytoplasm",
  "gene_symbol": "PDCL3",
  "gene_name": "Phosducin-like protein 3",
  "term_id": "GO:0005737"
}